active monoatomic ion transmembrane transporter activity [GO:0022853] (molecular function) Sources: GOC:mtg_transport, ISBN:0815340729 Also known as: active ion transmembrane transporter activity Definition: Enables the transfer of an ion from one side of a membrane to the other up the solute's concentration gradient. This is carried out by binding the solute and undergoing a series of conformational changes. Transport works equally well in either direction. Subtypes: cytochrome-c oxidase activity [GO:0004129], quinol-cytochrome-c reductase activity [GO:0008121], GO:0008137, proton-translocating NAD(P)+ transhydrogenase activity [GO:0008750], diphosphate hydrolysis-driven proton transmembrane transporter activity [GO:0009678], light-driven active monoatomic ion transmembrane transporter activity [GO:0015454], ATPase-coupled monoatomic cation transmembrane transporter activity [GO:0019829] Relationships: is a type of monoatomic ion transmembrane transporter activity [GO:0015075]; is a type of primary active transmembrane transporter activity [GO:0015399]